positive regulation of protein localization to cell cortex [GO:1904778] (biological process) Relationships: is a type of positive regulation of protein localization to cell periphery [GO:1904377]; is_a regulation of protein localization to cell cortex [GO:1904776]; positively regulates protein localization to cell cortex [GO:0072697] Note: An example is cye-1 in C. elegans, UniProt ID O01501 in PMID:17115027. References: PMID:17115027 Sources: GOC:TermGenie, GO_REF:0000058 Definition: Any process that activates or increases the frequency, rate or extent of protein localization to cell cortex. Also known as: positive regulation of protein localisation to cell cortex, up regulation of protein localisation to cell cortex, up regulation of protein localization to cell cortex, up-regulation of protein localisation to cell cortex, up-regulation of protein localization to cell cortex, upregulation of protein localisation to cell cortex, upregulation of protein localization to cell cortex, activation of protein localisation to cell cortex, activation of protein localization to cell cortex Subtypes: positive regulation of protein localization to medial cortex [GO:0106012], positive regulation of protein localization to actin cortical patch [GO:1904372]